{
  "term_id": "UNKNOWN:0001",
  "term_label": "Unknown molecular function",
  "gene": "UniProtKB:Q6MZQ0",
  "gene_name": "Proline-rich protein 5-like",
  "gene_symbol": "PRR5L"
}